detection of carbohydrate stimulus [GO:0009730] (biological process) Sources: GOC:sm Relationships: is a type of detection of chemical stimulus [GO:0009593]; is a type of response to carbohydrate [GO:0009743] Subtypes: detection of monosaccharide stimulus [GO:0034287], detection of disaccharide stimulus [GO:0034288] Definition: The series of events in which a carbohydrate stimulus is received by a cell and converted into a molecular signal. Also known as: perception of carbohydrate stimulus